{
  "term_label": "nucleus",
  "term_id": "GO:0005634",
  "gene": "UniProtKB:Q96PC2",
  "gene_name": "Inositol hexakisphosphate kinase 3",
  "gene_symbol": "IP6K3"
}